{
  "gene_symbol": "IGLV11-55",
  "gene_name": "Probable non-functional immunoglobulin lambda variable 11-55",
  "term_id": "GO:0006955",
  "term_label": "immune response",
  "gene": "UniProtKB:A0A075B6I3"
}